positive regulation of antigen processing and presentation of peptide antigen via MHC class I [GO:0002591] (biological process) Subtypes: positive regulation of antigen processing and presentation of endogenous peptide antigen via MHC class I [GO:1904284] Also known as: positive regulation of peptide antigen processing and presentation via MHC class I, up regulation of antigen processing and presentation of peptide antigen via MHC class I, up-regulation of antigen processing and presentation of peptide antigen via MHC class I, upregulation of antigen processing and presentation of peptide antigen via MHC class I, activation of antigen processing and presentation of peptide antigen via MHC class I, stimulation of antigen processing and presentation of peptide antigen via MHC class I Relationships: is a type of GO:0002585; is a type of regulation of antigen processing and presentation of peptide antigen via MHC class I [GO:0002589]; positively regulates antigen processing and presentation of peptide antigen via MHC class I [GO:0002474] Definition: Any process that activates or increases the frequency, rate, or extent of antigen processing and presentation of peptide antigen via MHC class I. Sources: GOC:add